{
  "gene_symbol": "LONP1",
  "gene_name": "Lon protease homolog, mitochondrial",
  "term_label": "ATP-dependent peptidase activity",
  "gene": "UniProtKB:P36776",
  "term_id": "GO:0004176"
}